{
  "gene": "UniProtKB:Q03135",
  "term_id": "GO:0048471",
  "gene_symbol": "CAV1",
  "term_label": "perinuclear region of cytoplasm",
  "gene_name": "Caveolin-1"
}